{
  "gene_name": "Tetratricopeptide repeat protein 16",
  "term_id": "UNKNOWN:0002",
  "term_label": "Unknown biological process",
  "gene_symbol": "TTC16",
  "gene": "UniProtKB:Q8NEE8"
}